{
  "term_label": "receptor complex",
  "gene_symbol": "GPRC5A",
  "gene_name": "Retinoic acid-induced protein 3",
  "gene": "UniProtKB:Q8NFJ5",
  "term_id": "GO:0043235"
}